{
  "term_label": "Unknown molecular function",
  "gene_symbol": "BID",
  "gene_name": "BH3-interacting domain death agonist",
  "term_id": "UNKNOWN:0001",
  "gene": "UniProtKB:P55957"
}